{
  "gene_symbol": "TGM6",
  "gene_name": "Protein-glutamine gamma-glutamyltransferase 6",
  "term_label": "peptide cross-linking",
  "term_id": "GO:0018149",
  "gene": "UniProtKB:O95932"
}